neurokinin receptor binding [GO:0031834] (molecular function) Also known as: neurokinin receptor ligand Relationships: is a type of neuropeptide receptor binding [GO:0071855] Subtypes: substance P receptor binding [GO:0031835], neuromedin K receptor binding [GO:0031836], substance K receptor binding [GO:0031837] Sources: GOC:mah, GOC:nln Definition: Binding to a neurokinin receptor.